{
  "gene_name": "Synaptonemal complex central element protein 3",
  "gene_symbol": "SYCE3",
  "gene": "UniProtKB:A1L190",
  "term_label": "central element",
  "term_id": "GO:0000801"
}